lysine carbamoyltransferase activity [GO:0050068] (molecular function) Relationships: is_a carboxyl- or carbamoyltransferase activity [GO:0016743] Definition: Catalysis of the reaction: L-lysine + carbamoyl phosphate = L-homocitrulline + H+ + phosphate. Also known as: carbamoyl-phosphate:L-lysine carbamoyltransferase activity, lysine transcarbamylase activity Sources: EC:2.1.3.8, RHEA:17121